{
  "term_id": "UNKNOWN:0001",
  "gene_symbol": "FNDC11",
  "gene": "UniProtKB:Q9BVV2",
  "gene_name": "Fibronectin type III domain-containing protein 11",
  "term_label": "Unknown molecular function"
}